{
  "gene": "UniProtKB:Q13635",
  "gene_name": "Protein patched homolog 1",
  "term_id": "GO:0097108",
  "gene_symbol": "PTCH1",
  "term_label": "hedgehog family protein binding"
}